regulation of maintenance of sister chromatid cohesion [GO:0034091] (biological process) Relationships: is a type of regulation of sister chromatid cohesion [GO:0007063]; regulates maintenance of sister chromatid cohesion [GO:0034086] Definition: Any process that modulates the extent to which the association between sister chromatids of a replicated chromosome is maintained. Subtypes: GO:0034092, GO:0034093, regulation of maintenance of meiotic sister chromatid cohesion [GO:0034094], GO:0034182 Sources: GOC:mah, GOC:vw